{
  "gene_symbol": "GPR107",
  "gene_name": "Protein GPR107",
  "term_id": "GO:0016020",
  "gene": "UniProtKB:Q5VW38",
  "term_label": "membrane"
}